{
  "gene_name": "Major vault protein",
  "gene": "UniProtKB:Q14764",
  "gene_symbol": "MVP",
  "term_id": "GO:0005737",
  "term_label": "cytoplasm"
}